SCF-Cdc4 ubiquitin ligase complex [GO:0097660] (cellular component) Relationships: is a type of SCF ubiquitin ligase complex [GO:0019005] Definition: An SCF ubiquitin ligase complex in which the F-box protein is Cdc4 in S. cerevisiae. References: PMID:9346238 Sources: GOC:jd, GOC:vw